{
  "gene_name": "Flotillin-2",
  "term_label": "protein localization to plasma membrane",
  "gene": "UniProtKB:Q14254",
  "gene_symbol": "FLOT2",
  "term_id": "GO:0072659"
}